{
  "term_label": "bile acid transmembrane transporter activity",
  "gene_name": "Solute carrier organic anion transporter family member 1C1",
  "term_id": "GO:0015125",
  "gene_symbol": "SLCO1C1",
  "gene": "UniProtKB:Q9NYB5"
}